{
  "gene": "UniProtKB:Q9NR19",
  "gene_name": "Acetyl-coenzyme A synthetase, cytoplasmic",
  "term_id": "GO:0006085",
  "term_label": "acetyl-CoA biosynthetic process",
  "gene_symbol": "ACSS2"
}